{
  "gene_name": "Putative uncharacterized protein LQK1",
  "term_id": "UNKNOWN:0002",
  "gene": "UniProtKB:Q8TAF5",
  "term_label": "Unknown biological process",
  "gene_symbol": "FLVCR1-DT"
}